{
  "gene_symbol": "SIX1",
  "gene_name": "Homeobox protein SIX1",
  "gene": "UniProtKB:Q15475",
  "term_label": "transcription regulator complex",
  "term_id": "GO:0005667"
}